{
  "term_id": "UNKNOWN:0003",
  "gene_symbol": "ENPP7",
  "gene_name": "Ectonucleotide pyrophosphatase_phosphodiesterase family member 7",
  "term_label": "Unknown cellular component",
  "gene": "UniProtKB:Q6UWV6"
}